{
  "gene": "UniProtKB:Q15059",
  "gene_symbol": "BRD3",
  "term_label": "regulation of transcription by RNA polymerase II",
  "gene_name": "Bromodomain-containing protein 3",
  "term_id": "GO:0006357"
}